response to jasmonic acid [GO:0009753] (biological process) Definition: Any process that results in a change in state or activity of a cell or an organism (in terms of movement, secretion, enzyme production, gene expression, etc.) as a result of a jasmonic acid stimulus. Sources: GOC:jl Also known as: response to jasmonic acid stimulus Relationships: is a type of response to hormone [GO:0009725]; is a type of response to fatty acid [GO:0070542] Subtypes: detection of jasmonic acid stimulus [GO:0009754], response to jasmonic acid stimulus involved in jasmonic acid and ethylene-dependent systemic resistance [GO:0032260], cellular response to jasmonic acid stimulus [GO:0071395]